{
  "gene_name": "Neutral amino acid transporter B(0)",
  "term_label": "plasma membrane",
  "gene": "UniProtKB:Q15758",
  "gene_symbol": "SLC1A5",
  "term_id": "GO:0005886"
}